{
  "gene_symbol": "STOM",
  "gene": "UniProtKB:P27105",
  "term_id": "GO:0008200",
  "gene_name": "Stomatin",
  "term_label": "ion channel inhibitor activity"
}